{
  "gene_name": "Tektin-3",
  "gene_symbol": "TEKT3",
  "term_id": "GO:0060294",
  "gene": "UniProtKB:Q9BXF9",
  "term_label": "cilium movement involved in cell motility"
}